L-tryptophan catabolic process to catechol [GO:0019444] (BP) Also known as: tryptophan breakdown to catechol, tryptophan catabolic process to catechol, tryptophan degradation to catechol Sources: GOC:go_curators Definition: The chemical reactions and pathways resulting in the breakdown of L-tryptophan into other compounds, including catechol. Relationships: is a type of GO:0006569; is a type of catechol-containing compound metabolic process [GO:0009712]